diphosphoinositol polyphosphate catabolic process [GO:0071544] (biological process) Definition: The chemical reactions and pathways resulting in the breakdown of a diphosphoinositol polyphosphate, 1,2,3,4,5,6-cyclohexanehexol with one or more diphosphate groups and multiple monophosphate groups attached. References: PMID:12387729 Sources: GOC:mah Also known as: diphosphoinositol polyphosphate breakdown, diphosphoinositol polyphosphate catabolism, diphosphoinositol polyphosphate degradation Relationships: is a type of GO:0071543; is a type of inositol phosphate catabolic process [GO:0071545]